Ragulator complex [GO:0071986] (cellular component) Definition: A vacuolar membrane-anchored guanine nucleotide exchange factor (GEF) complex for the Rag GTPases (Gtr1-Gtr2 GTPase complex GO:1990131) in TORC1 signaling pathway. In human, Ragulator is comprised of the membrane anchor subunit LAMTOR1 (Meh1p in S. cerevisiae, Lam1 in S. pombe), a GEF subunit LAMTOR2 ( Slm4 in S. cerevisiae , Lam2 in S. pombe ) , LAMTOR3 (no S. cerevisiae ortholog identified, Lam3 in S. pombe) , LAMTOR4 (no S. cerevisiae ortholog identified, Lam4 in S. pombe), and LAMTOR5 (no S. cerevisiae or S. pombe ortholog identified). References: PMID:15989961, PMID:16732272, PMID:19177150, PMID:19748353, PMID:20381137, PMID:22980980, PMID:29199950 Sources: GOC:vw Also known as: MAPKSP1/ROBLD3/C11orf59 complex, Rag GEF, EGO complex, EGO-GSE complex, GSE complex, GTPase-containing complex for Gap1p sorting in the endosome Relationships: is a type of guanyl-nucleotide exchange factor complex [GO:0032045]; is a type of membrane protein complex [GO:0098796]; is part of GO:0005774